mitochondrial cysteinyl-tRNA aminoacylation [GO:0070147] (biological process) Definition: The process of coupling cysteine to cysteinyl-tRNA in a mitochondrion, catalyzed by cysteinyl-tRNA synthetase. In tRNA aminoacylation, the amino acid is first activated by linkage to AMP and then transferred to either the 2'- or the 3'-hydroxyl group of the 3'-adenosine residue of the tRNA. Relationships: is a type of cysteinyl-tRNA aminoacylation [GO:0006423]; is a type of tRNA aminoacylation for mitochondrial protein translation [GO:0070127] Sources: GOC:mah, GOC:mcc